{
  "term_id": "GO:0071577",
  "gene_name": "Probable proton-coupled zinc antiporter SLC30A4",
  "term_label": "zinc ion transmembrane transport",
  "gene": "UniProtKB:O14863",
  "gene_symbol": "SLC30A4"
}